endopolyphosphatase activity [GO:0000298] (molecular function) Relationships: is a type of pyrophosphatase activity [GO:0016462] Sources: EC:3.6.1.10 Definition: Catalysis of the reaction: polyphosphate + n H2O = (n+1) oligophosphate. The product contains 4 or 5 phosphate residues. Also known as: metaphosphatase activity, polyphosphatase activity, polyphosphate depolymerase activity, polymetaphosphatase activity, polyphosphate polyphosphohydrolase activity